{
  "gene": "UniProtKB:Q6P5X5",
  "term_label": "Unknown cellular component",
  "gene_name": "UPF0545 protein C22orf39",
  "gene_symbol": "C22orf39",
  "term_id": "UNKNOWN:0003"
}